{
  "gene": "UniProtKB:Q9UKJ8",
  "term_label": "external side of plasma membrane",
  "gene_symbol": "ADAM21",
  "term_id": "GO:0009897",
  "gene_name": "Disintegrin and metalloproteinase domain-containing protein 21"
}